RNA polymerase II C-terminal domain S5 O-GlcNAc transferase activity [GO:0140842] (molecular function) Relationships: is a type of GO:0140841 Definition: Catalysis of the reaction: UDP-N-acetyl-D-glucosamine + RNA polymerase II large subunit CTD heptapeptide repeat (YSPTSPS) = UDP + RNA polymerase II large subunit CTD heptapeptide repeat 3-O-(N-acetyl-D-glucosaminyl)-L-serine (position 5). References: PMID:22605332